{
  "term_label": "GTPase activity",
  "gene_name": "Septin-2",
  "term_id": "GO:0003924",
  "gene_symbol": "SEPTIN2",
  "gene": "UniProtKB:Q15019"
}